sphingolipid mediated signaling pathway [GO:0090520] (biological process) Definition: The series of molecular signals mediated by a sphingolipid. References: PMID:9525917 Also known as: sphingolipid mediated signal transduction, sphingolipid-mediated signaling pathway, ceramide 1-phosphate signaling pathway, ceramide signaling pathway, sphingosine signaling pathway, sphingolipid signaling pathway Relationships: is a type of GO:0007165 Subtypes: sphingosine-1-phosphate receptor signaling pathway [GO:0003376] Regulation: regulated by regulation of sphingolipid mediated signaling pathway [GO:1902068]; negatively regulated by negative regulation of sphingolipid mediated signaling pathway [GO:1902069]; positively regulated by positive regulation of sphingolipid mediated signaling pathway [GO:1902070]